{
  "gene_symbol": "HYCC1",
  "gene_name": "Hyccin",
  "term_id": "GO:0005886",
  "term_label": "plasma membrane",
  "gene": "UniProtKB:Q9BYI3"
}